negative regulation of retrograde transport, endosome to Golgi [GO:1905280] (biological process) Also known as: down regulation of retrograde (endosome to Golgi) transport, down regulation of retrograde transport, endosome to Golgi, down-regulation of retrograde (endosome to Golgi) transport, down-regulation of retrograde transport, endosome to Golgi, downregulation of retrograde (endosome to Golgi) transport, downregulation of retrograde transport, endosome to Golgi, negative regulation of retrograde (endosome to Golgi) transport, inhibition of retrograde (endosome to Golgi) transport, inhibition of retrograde transport, endosome to Golgi Definition: Any process that stops, prevents or reduces the frequency, rate or extent of retrograde transport, endosome to Golgi. Relationships: is a type of GO:0032387; is a type of regulation of retrograde transport, endosome to Golgi [GO:1905279]; negatively regulates GO:0042147 Sources: GOC:PARL, GOC:TermGenie, GOC:bf, GO_REF:0000058